response to redox state [GO:0051775] (biological process) Definition: Any process that results in a change in state or activity of a cell or an organism (in terms of movement, secretion, enzyme production, gene expression, etc.) as a result of a stimulus indicating redox state. Redox state refers to the balance of oxidized versus reduced forms of electron donors and acceptors in an organelle, cell or organ; plastoquinone, glutathione (GSH/GSSG), and nicotinamide nucleotides (NAD+/NADH and NADP+/NADPH) are among the most important. Relationships: is a type of response to stimulus [GO:0050896] Also known as: redox signal response References: PMID:15131240, PMID:16987039 Sources: GOC:mah Subtypes: redox taxis [GO:0009455], detection of redox state [GO:0051776], cellular response to redox state [GO:0071461]